D-cysteine catabolic process [GO:0019447] (biological process) References: PMID:11527960 Relationships: is a type of cysteine catabolic process [GO:0009093]; is a type of D-amino acid catabolic process [GO:0019478] Also known as: D-cysteine breakdown, D-cysteine catabolism, D-cysteine degradation Definition: The chemical reactions and pathways resulting in the breakdown of D-cysteine, (S)-2-amino-3-mercaptopropanoic acid, which occurs naturally in firefly luciferin.